indoleacetaldoxime dehydratase activity [GO:0047720] (molecular function) Definition: Catalysis of the reaction: (indol-3-yl)acetaldehyde oxime = (indol-3-yl)acetonitrile + H2O. Sources: RHEA:23156 Also known as: (indol-3-yl)acetaldehyde-oxime hydro-lyase activity, 3-indoleacetaldoxime hydro-lyase activity, indole-3-acetaldehyde-oxime hydro-lyase activity, indole-3-acetaldoxime hydro-lyase activity, indoleacetaldoxime hydro-lyase activity Relationships: is a type of GO:0141122